mitochondrial pyruvate carrier complex [GO:7770001] (cellular component) References: PMID:22628554, PMID:22628558 Relationships: is a type of inner mitochondrial membrane protein complex [GO:0098800]; is a type of transmembrane transporter complex [GO:1902495] Definition: An inner mitochondrial protein carrier capable of transporting pyruvate into the mitochondrion.